{
  "term_label": "ubiquitin-ubiquitin ligase activity",
  "gene_symbol": "UBR5",
  "gene": "UniProtKB:O95071",
  "term_id": "GO:0034450",
  "gene_name": "E3 ubiquitin-protein ligase UBR5"
}